{
  "term_id": "GO:0043161",
  "term_label": "proteasome-mediated ubiquitin-dependent protein catabolic process",
  "gene_name": "Gigaxonin",
  "gene_symbol": "GAN",
  "gene": "UniProtKB:Q9H2C0"
}